{
  "term_label": "Unknown molecular function",
  "gene_name": "Uncharacterized protein DKFZp781C0719",
  "gene_symbol": "DKFZp781C0719",
  "term_id": "UNKNOWN:0001",
  "gene": "UniProtKB:Q68DW6"
}